{
  "gene_name": "Lysozyme-like protein 6",
  "term_label": "fusion of sperm to egg plasma membrane involved in single fertilization",
  "term_id": "GO:0007342",
  "gene_symbol": "LYZL6",
  "gene": "UniProtKB:O75951"
}